{
  "gene_name": "Isoamyl acetate-hydrolyzing esterase 1 homolog",
  "term_id": "GO:0016788",
  "gene_symbol": "IAH1",
  "term_label": "hydrolase activity, acting on ester bonds",
  "gene": "UniProtKB:Q2TAA2"
}